{
  "gene_name": "Beta-nerve growth factor",
  "gene_symbol": "NGF",
  "term_label": "negative regulation of neuron apoptotic process",
  "gene": "UniProtKB:P01138",
  "term_id": "GO:0043524"
}